{
  "term_id": "GO:0008510",
  "gene_name": "Sodium-driven chloride bicarbonate exchanger",
  "gene_symbol": "SLC4A10",
  "term_label": "sodium:bicarbonate symporter activity",
  "gene": "UniProtKB:Q6U841"
}